{
  "gene_name": "Zinc-activated ligand-gated ion channel",
  "term_id": "UNKNOWN:0001",
  "gene_symbol": "ZACN",
  "term_label": "Unknown molecular function",
  "gene": "UniProtKB:Q401N2"
}